{
  "term_label": "U2 snRNA binding",
  "term_id": "GO:0030620",
  "gene_name": "U2 small nuclear ribonucleoprotein A'",
  "gene": "UniProtKB:P09661",
  "gene_symbol": "SNRPA1"
}